perinucleolar chromocenter [GO:0010370] (cellular component) Definition: A chromocenter adjacent to the nucleolus. References: PMID:15805479 Relationships: is a type of GO:0010369